coniferyl-aldehyde dehydrogenase [NAD(P)+] activity [GO:0050269] (molecular function) Definition: Catalysis of the reaction: coniferyl aldehyde + H2O + NAD(P)+ = ferulate + NAD(P)H + H+. Relationships: is a type of GO:0004030 Sources: EC:1.2.1.68 Also known as: coniferyl aldehyde:NAD(P)+ oxidoreductase activity